regulation of mitochondrial ATP synthesis coupled proton transport [GO:1905706] (biological process) Subtypes: negative regulation of mitochondrial ATP synthesis coupled proton transport [GO:1905707] Relationships: is a type of GO:2001169; regulates GO:0042776 Definition: Any process that modulates the frequency, rate or extent of mitochondrial ATP synthesis coupled proton transport. References: PMID:12809520, PMID:15294286 Sources: GOC:TermGenie, GO_REF:0000058